{
  "gene": "UniProtKB:Q9H4K7",
  "term_id": "GO:0005525",
  "gene_symbol": "MTG2",
  "term_label": "GTP binding",
  "gene_name": "Mitochondrial ribosome-associated GTPase 2"
}